{
  "term_label": "Unknown molecular function",
  "gene": "UniProtKB:Q9H4G1",
  "gene_symbol": "CST9L",
  "term_id": "UNKNOWN:0001",
  "gene_name": "Cystatin-9-like"
}